{
  "term_id": "UNKNOWN:0002",
  "gene": "UniProtKB:A0A1B0GU71",
  "gene_symbol": "CFAP97D2",
  "term_label": "Unknown biological process",
  "gene_name": "Uncharacterized protein CFAP97D2"
}